{
  "gene_symbol": "POLE4",
  "gene": "UniProtKB:Q9NR33",
  "term_id": "GO:0008622",
  "term_label": "epsilon DNA polymerase complex",
  "gene_name": "DNA polymerase epsilon subunit 4"
}